{
  "gene": "UniProtKB:P07438",
  "gene_symbol": "MT1B",
  "term_id": "GO:0071280",
  "term_label": "cellular response to copper ion",
  "gene_name": "Metallothionein-1B"
}